{
  "gene": "UniProtKB:P0C851",
  "gene_symbol": "PIRT",
  "term_label": "plasma membrane",
  "term_id": "GO:0005886",
  "gene_name": "Phosphoinositide-interacting protein"
}